Delta4-3-oxosteroid 5beta-reductase activity [GO:0047787] (molecular function) Sources: EC:1.3.1.3 Also known as: 5-beta-reductase activity, 3-oxo-5beta-steroid:NADP+ delta4-oxidoreductase activity, 3-oxo-Delta(4)-steroid 5-beta-reductase activity, 3-oxo-Delta4-steroid 5beta-reductase activity, Delta4-3-oxosteroid 5-beta-reductase activity, 4,5beta-dihydrocortisone:NADP+ delta4-oxidoreductase activity, 5beta-cholestan-3-one:NADP+ 4,5-oxidoreductase activity, androstenedione 5-beta-reductase activity, androstenedione 5beta-reductase activity, cholestenone 5-beta-reductase activity, cholestenone 5b-reductase activity, cholestenone 5beta-reductase activity, cortisone 5-beta-reductase activity, cortisone 5beta-reductase activity, cortisone b-reductase activity, cortisone beta-reductase activity, cortisone delta(4)-5-beta-reductase activity, testosterone 5-beta-reductase activity, testosterone 5beta-reductase activity, 5beta-reductase activity, Delta(4)-3-ketosteroid 5-beta-reductase activity, Delta(4)-5-beta-reductase activity, Delta(4)-hydrogenase activity, Delta4-3-ketosteroid 5beta-reductase activity, Delta4-5beta-reductase activity, Delta4-hydrogenase activity, cortisone delta4-5beta-reductase activity, steroid 5-beta-reductase activity, steroid 5beta-reductase activity Definition: Catalysis of the reaction: a 3-oxo-5beta-steroid + NADP+ = a 3-oxo-Delta(4)-steroid + H+ + NADPH. The enzyme from human efficiently catalyzes the reduction of progesterone, androstenedione, 17alpha-hydroxyprogesterone and testosterone to 5beta-reduced metabolites; it can also act on aldosterone, corticosterone and cortisol, but to a lesser extent. The bile acid intermediates 7alpha,12alpha-dihydroxy-4-cholesten-3- one and 7alpha-hydroxy-4-cholesten-3-one can also act as substrates. Relationships: is a type of enone reductase activity [GO:0035671]